{
  "gene_name": "Zinc finger MYM-type protein 5",
  "gene_symbol": "ZMYM5",
  "term_id": "UNKNOWN:0001",
  "gene": "UniProtKB:Q9UJ78",
  "term_label": "Unknown molecular function"
}